cysteine biosynthetic process via S-sulfo-L-cysteine [GO:0019345] (biological process) Also known as: cysteine anabolism via S-sulfo-L-cysteine, cysteine biosynthesis via S-sulpho-L-cysteine, cysteine biosynthetic process via S-sulpho-L-cysteine, cysteine formation via S-sulfo-L-cysteine, cysteine synthesis via S-sulfo-L-cysteine Definition: The chemical reactions and pathways resulting in the formation of cysteine, via the intermediate S-sulfo-L-cysteine. Relationships: is_a GO:0019344 Sources: GOC:go_curators